protein-N(PI)-phosphohistidine-glucose phosphotransferase system transporter activity [GO:0022855] (molecular function) Definition: Catalysis of the PEP-dependent, phosphoryl transfer-driven transport of substances across a membrane. The transport happens by catalysis of the reaction: protein N-phosphohistidine + glucose(out) = protein histidine + glucose phosphate(in). This differs from primary and secondary active transport in that the solute is modified during transport. Relationships: is a type of protein-N(PI)-phosphohistidine-sugar phosphotransferase activity [GO:0008982]; is a type of D-glucose transmembrane transporter activity [GO:0055056] Also known as: glucose PTS transporter activity Sources: GOC:mtg_transport, ISBN:0815340729